{
  "gene_name": "Glutathione peroxidase 1",
  "gene_symbol": "GPX1",
  "gene": "UniProtKB:P07203",
  "term_label": "cellular response to oxidative stress",
  "term_id": "GO:0034599"
}